{
  "gene_name": "Maturin",
  "gene": "UniProtKB:Q8N3F0",
  "term_label": "cytoplasm",
  "gene_symbol": "MTURN",
  "term_id": "GO:0005737"
}